{
  "gene_symbol": "ITGB2",
  "gene": "UniProtKB:P05107",
  "term_id": "GO:0030593",
  "gene_name": "Integrin beta-2",
  "term_label": "neutrophil chemotaxis"
}